{
  "term_id": "GO:0001919",
  "term_label": "regulation of receptor recycling",
  "gene": "UniProtKB:Q6IAA8",
  "gene_symbol": "LAMTOR1",
  "gene_name": "Ragulator complex protein LAMTOR1"
}